{
  "term_label": "N-acetyl-L-aspartate-L-glutamate ligase activity",
  "gene_name": "Beta-citrylglutamate synthase B",
  "gene_symbol": "RIMKLB",
  "gene": "UniProtKB:Q9ULI2",
  "term_id": "GO:0072590"
}